{
  "gene_symbol": "EDN3",
  "term_id": "GO:0003100",
  "term_label": "regulation of systemic arterial blood pressure by endothelin",
  "gene": "UniProtKB:P14138",
  "gene_name": "Endothelin-3"
}